{
  "term_id": "UNKNOWN:0002",
  "gene": "UniProtKB:Q9NWH2",
  "gene_name": "Transmembrane protein 242",
  "term_label": "Unknown biological process",
  "gene_symbol": "TMEM242"
}